{
  "gene_symbol": "PLXNA3",
  "term_id": "GO:0071526",
  "gene_name": "Plexin-A3",
  "term_label": "semaphorin-plexin signaling pathway",
  "gene": "UniProtKB:P51805"
}